ficolin-1-rich granule [GO:0101002] (cellular component) Also known as: ficolin-1 rich granule, ficolin granule Definition: Highly exocytosable gelatinase-poor granules found in neutrophils and rich in ficolin-1. Ficolin-1 is released from neutrophil granules by stimulation with fMLP or PMA, and the majority becomes associated with the surface membrane of the cells and can be detected by flow cytometry. Relationships: is_a secretory granule [GO:0030141] References: PMID:19741154 Sources: GOC:mec